{
  "term_id": "GO:0016064",
  "gene_name": "Immunoglobulin heavy variable 3-49",
  "gene": "UniProtKB:A0A0A0MS15",
  "gene_symbol": "IGHV3-49",
  "term_label": "immunoglobulin mediated immune response"
}